{
  "gene": "UniProtKB:P19256",
  "gene_symbol": "CD58",
  "term_label": "immune response",
  "gene_name": "Lymphocyte function-associated antigen 3",
  "term_id": "GO:0006955"
}